{
  "gene": "UniProtKB:O75312",
  "gene_symbol": "ZPR1",
  "term_id": "GO:0010628",
  "term_label": "positive regulation of gene expression",
  "gene_name": "Zinc finger protein ZPR1"
}